{
  "gene_name": "Tyrosine-protein kinase ITK_TSK",
  "term_id": "GO:0001865",
  "gene_symbol": "ITK",
  "term_label": "NK T cell differentiation",
  "gene": "UniProtKB:Q08881"
}